endoplasmic reticulum-Golgi intermediate compartment [GO:0005793] (cellular component) References: PMID:16723730 Sources: GOC:pr Definition: A complex system of membrane-bounded compartments located between endoplasmic reticulum (ER) and the Golgi complex, with a distinctive membrane protein composition; involved in ER-to-Golgi and Golgi-to-ER transport. Relationships: is a type of intracellular membrane-bounded organelle [GO:0043231]; is part of cytoplasm [GO:0005737] Also known as: EGTC, ER-Golgi intermediate compartment, ER-Golgi transport container, ERGIC, VTC, endoplasmic reticulum-Golgi transport container, pre-Golgi intermediate compartment, vesicular-tubular cluster